{
  "term_id": "UNKNOWN:0001",
  "gene_name": "Nucleolar pre-ribosomal-associated protein 1",
  "gene_symbol": "URB1",
  "gene": "UniProtKB:O60287",
  "term_label": "Unknown molecular function"
}